{
  "gene_name": "Intestinal-type alkaline phosphatase",
  "term_id": "UNKNOWN:0002",
  "gene": "UniProtKB:P09923",
  "gene_symbol": "ALPI",
  "term_label": "Unknown biological process"
}